{
  "gene_symbol": "ROR1",
  "term_id": "GO:0043123",
  "gene": "UniProtKB:Q01973",
  "gene_name": "Inactive tyrosine-protein kinase transmembrane receptor ROR1",
  "term_label": "positive regulation of canonical NF-kappaB signal transduction"
}